{
  "term_id": "GO:0035556",
  "term_label": "intracellular signal transduction",
  "gene": "UniProtKB:Q9H9S4",
  "gene_name": "Calcium-binding protein 39-like",
  "gene_symbol": "CAB39L"
}